{
  "term_id": "GO:0006612",
  "gene": "UniProtKB:Q6UX98",
  "gene_name": "Probable palmitoyltransferase ZDHHC24",
  "term_label": "protein targeting to membrane",
  "gene_symbol": "ZDHHC24"
}